{
  "gene": "UniProtKB:P08861",
  "gene_name": "Chymotrypsin-like elastase family member 3B",
  "term_label": "extracellular space",
  "gene_symbol": "CELA3B",
  "term_id": "GO:0005615"
}